{
  "gene": "UniProtKB:A0MZ66",
  "term_id": "GO:0048812",
  "gene_name": "Shootin-1",
  "gene_symbol": "SHTN1",
  "term_label": "neuron projection morphogenesis"
}